{
  "gene": "UniProtKB:Q8WXX5",
  "gene_symbol": "DNAJC9",
  "term_id": "UNKNOWN:0002",
  "term_label": "Unknown biological process",
  "gene_name": "DnaJ homolog subfamily C member 9"
}